high-affinity secondary active nitrite transmembrane transporter activity [GO:0015513] (molecular function) Relationships: is a type of nitrate transmembrane transporter activity [GO:0015112]; is a type of secondary active transmembrane transporter activity [GO:0015291] Subtypes: nitrate:proton symporter activity [GO:0009671], nitrate efflux transmembrane transporter activity [GO:0010542] Also known as: nitrite uptake permease activity Sources: GOC:mtg_transport, ISBN:0815340729 Definition: Catalysis of the transfer of nitrite from one side of the membrane to the other, up the solute's concentration gradient. The transporter binds the solute and undergoes a series of conformational changes. Transport works equally well in either direction and is driven by a chemiosmotic source of energy. In high affinity transport the transporter is able to bind the solute even if it is only present at very low concentrations.